{
  "term_id": "GO:0070588",
  "gene": "UniProtKB:Q9UBN4",
  "gene_symbol": "TRPC4",
  "term_label": "calcium ion transmembrane transport",
  "gene_name": "Short transient receptor potential channel 4"
}